3-dehydroquinate synthase activity [GO:0003856] (molecular function) Definition: Catalysis of the reaction: 7-phospho-2-dehydro-3-deoxy-D-arabino-heptonate = 3-dehydroquinate + phosphate. Sources: EC:4.2.3.4, RHEA:21968 Relationships: is a type of carbon-oxygen lyase activity, acting on phosphates [GO:0016838]